lobar bronchus development [GO:0060482] (biological process) Relationships: is a type of GO:0060433 Definition: The biological process whose specific outcome is the progression of a lobar bronchus from an initial condition to its mature state. This process begins with the formation of the lobar bronchus and ends with the mature structure. The lobar bronchus is the major airway within the respiratory tree that starts by division of the principal bronchi on both sides and ends at the point of its own subdivision into tertiary or segmental bronchi. Sources: GOC:dph, GOC:mtg_lung